agmatine biosynthetic process [GO:0097055] (biological process) Definition: The chemical reactions and pathways resulting in the formation of agmatine ((4-aminobutyl)guanidine, NH2-CH2-CH2-CH2-CH2-NH-C(-NH2)(=NH)). Agmatine is the decarboxylation product of the amino acid arginine and is an intermediate in polyamine biosynthesis. It is synthesized in the brain, stored in synaptic vesicles, accumulated by uptake, released by membrane depolarization, and inactivated by agmatinase. Sources: GOC:pr, GOC:yaf Also known as: agmatine anabolism, agmatine biosynthesis, agmatine formation, agmatine synthesis Relationships: is a type of GO:1901162